{
  "term_label": "G protein-coupled receptor signaling pathway",
  "term_id": "GO:0007186",
  "gene_symbol": "OR5M1",
  "gene": "UniProtKB:Q8NGP8",
  "gene_name": "Olfactory receptor 5M1"
}